Snt2C complex [GO:0070211] (cellular component) Relationships: is a type of histone deacetylase complex [GO:0000118]; is part of chromatin [GO:0000785] References: PMID:19040720 Sources: GOC:rb Definition: A histone deacetylase complex that is part of the chromatin remodeling machinery. In Saccharomyces cerevisiae this complex contains Snt2p, Ecm5p and Rpd3p.